{
  "gene": "UniProtKB:Q8WXE1",
  "gene_name": "ATR-interacting protein",
  "gene_symbol": "ATRIP",
  "term_id": "UNKNOWN:0003",
  "term_label": "Unknown cellular component"
}